regulation of xanthone-containing compound biosynthetic process [GO:1900183] (biological process) Definition: Any process that modulates the frequency, rate or extent of xanthone-containing compound biosynthetic process. Subtypes: negative regulation of xanthone-containing compound biosynthetic process [GO:1900184], positive regulation of xanthone-containing compound biosynthetic process [GO:1900185], regulation of emericellin biosynthetic process [GO:1900834] Also known as: regulation of xanthone-containing compound anabolism, regulation of xanthone-containing compound biosynthesis, regulation of xanthone-containing compound formation, regulation of xanthone-containing compound synthesis, regulation of xanthone biosynthesis, regulation of xanthone biosynthetic process Sources: GOC:TermGenie, GOC:di Relationships: is a type of regulation of ketone biosynthetic process [GO:0010566]; regulates xanthone-containing compound biosynthetic process [GO:2001307]